circulatory system development [GO:0072359] (biological process) Definition: The process whose specific outcome is the progression of the circulatory system over time, from its formation to the mature structure. The circulatory system is the organ system that passes nutrients (such as amino acids and electrolytes), gases, hormones, blood cells, etc. to and from cells in the body to help fight diseases and help stabilize body temperature and pH to maintain homeostasis. Also known as: cardiovascular system development Relationships: is a type of system development [GO:0048731] Sources: GOC:mah, UBERON:0001009